{
  "term_label": "positive regulation of cytoplasmic translation",
  "gene_symbol": "CNBP",
  "gene": "UniProtKB:P62633",
  "term_id": "GO:2000767",
  "gene_name": "CCHC-type zinc finger nucleic acid binding protein"
}